{
  "gene": "UniProtKB:P26038",
  "gene_symbol": "MSN",
  "gene_name": "Moesin",
  "term_id": "GO:0050839",
  "term_label": "cell adhesion molecule binding"
}